triterpenoid catabolic process [GO:0016105] (biological process) Sources: GOC:go_curators Relationships: is a type of triterpenoid metabolic process [GO:0006722]; is a type of terpenoid catabolic process [GO:0016115] Subtypes: GO:0010684, pentacyclic triterpenoid catabolic process [GO:0019741], hopanoid catabolic process [GO:0019743], (17Z)-protosta-17(20),24-dien-3beta-ol catabolic process [GO:1900580] Definition: The chemical reactions and pathways resulting in the breakdown of triterpenoid compounds, terpenoids with six isoprene units. Also known as: triterpenoid breakdown, triterpenoid catabolism, triterpenoid degradation, triterpene catabolic process, triterpene catabolism